{
  "gene": "UniProtKB:Q8WW14",
  "gene_name": "Uncharacterized protein C10orf82",
  "term_id": "UNKNOWN:0002",
  "term_label": "Unknown biological process",
  "gene_symbol": "C10orf82"
}